{
  "term_label": "neuron apoptotic process",
  "term_id": "GO:0051402",
  "gene": "UniProtKB:Q1L5Z9",
  "gene_symbol": "LONRF2",
  "gene_name": "LON peptidase N-terminal domain and RING finger protein 2"
}